smooth endoplasmic reticulum membrane [GO:0030868] (cellular component) Definition: The lipid bilayer surrounding the smooth endoplasmic reticulum. Relationships: is a type of endoplasmic reticulum membrane [GO:0005789]; is a type of bounding membrane of organelle [GO:0098588]; is part of smooth endoplasmic reticulum [GO:0005790] Also known as: SER membrane, smooth ER membrane Sources: GOC:mah